alphaIIb-beta3 integrin-CD47-Src complex [GO:0070771] (cellular component) Relationships: is a type of plasma membrane protein complex [GO:0098797] References: PMID:9169439 Definition: A protein complex that consists of an alphaIIb-beta3 integrin complex bound to the cell surface antigen CD47 and the kinase c-Src. Also known as: ITGA2b-ITGB3-CD47-SRC complex